endocrocin catabolic process [GO:1900601] (biological process) Relationships: is a type of phenol-containing compound catabolic process [GO:0019336]; is a type of ketone catabolic process [GO:0042182]; is_a carboxylic acid catabolic process [GO:0046395]; is a type of secondary metabolite catabolic process [GO:0090487] Sources: GOC:TermGenie, GOC:di Also known as: endocrocin breakdown, endocrocin catabolism, endocrocin degradation Definition: The chemical reactions and pathways resulting in the breakdown of endocrocin.